{
  "gene": "UniProtKB:Q6DD87",
  "term_label": "DNA-binding transcription factor activity, RNA polymerase II-specific",
  "term_id": "GO:0000981",
  "gene_symbol": "ZNF787",
  "gene_name": "Zinc finger protein 787"
}